female germline ring canal formation, actin assembly [GO:0008302] (biological process) Also known as: ring canal formation, actin assembly, nurse cell ring canal formation, actin assembly, ovarian ring canal formation, actin assembly Definition: Recruitment and organization of actin filaments in female germline ring canals. Sources: ISBN:0879694238 Relationships: is a type of actin filament organization [GO:0007015]; is part of female germline ring canal formation [GO:0007301]